{
  "gene_symbol": "DNAJC11",
  "term_id": "UNKNOWN:0001",
  "gene": "UniProtKB:Q9NVH1",
  "gene_name": "DnaJ homolog subfamily C member 11",
  "term_label": "Unknown molecular function"
}